{
  "term_label": "acetylcholine receptor regulator activity",
  "gene_symbol": "AGRN",
  "gene": "UniProtKB:O00468",
  "term_id": "GO:0030548",
  "gene_name": "Agrin"
}